benzoate transport [GO:0042919] (biological process) Definition: The directed movement of benzoate, the anion of benzoic acid (benzenecarboxylic acid) into, out of or within a cell, or between cells, by means of some agent such as a transporter or pore. Relationships: is a type of monocarboxylic acid transport [GO:0015718] Sources: GOC:jl, ISBN:0721662544